{
  "gene_name": "Nostrin",
  "gene": "UniProtKB:Q8IVI9",
  "term_label": "Unknown biological process",
  "gene_symbol": "NOSTRIN",
  "term_id": "UNKNOWN:0002"
}